{
  "gene_symbol": "PSME3IP1",
  "gene": "UniProtKB:Q9GZU8",
  "term_id": "UNKNOWN:0002",
  "term_label": "Unknown biological process",
  "gene_name": "PSME3-interacting protein"
}